{
  "gene_symbol": "CMTR1",
  "term_label": "nucleus",
  "term_id": "GO:0005634",
  "gene": "UniProtKB:Q8N1G2",
  "gene_name": "Cap-specific mRNA (nucleoside-2'-O-)-methyltransferase 1"
}